{
  "gene_name": "Uncharacterized protein C6orf136",
  "term_id": "UNKNOWN:0002",
  "gene_symbol": "C6orf136",
  "term_label": "Unknown biological process",
  "gene": "UniProtKB:Q5SQH8"
}